{
  "gene": "UniProtKB:P48378",
  "term_id": "GO:0060271",
  "gene_name": "DNA-binding protein RFX2",
  "term_label": "cilium assembly",
  "gene_symbol": "RFX2"
}